interleukin-6 receptor binding [GO:0005138] (molecular function) Sources: GOC:ai Definition: Binding to an interleukin-6 receptor. Relationships: is a type of cytokine receptor binding [GO:0005126]; is a type of growth factor receptor binding [GO:0070851] Also known as: IL-6, interleukin-6 receptor ligand